{
  "term_id": "GO:0005829",
  "term_label": "cytosol",
  "gene_name": "AP-5 complex subunit sigma-1",
  "gene_symbol": "AP5S1",
  "gene": "UniProtKB:Q9NUS5"
}